{
  "term_id": "GO:0097602",
  "term_label": "cullin family protein binding",
  "gene": "UniProtKB:Q9BTE7",
  "gene_name": "DCN1-like protein 5",
  "gene_symbol": "DCUN1D5"
}